{
  "term_label": "olfactory receptor activity",
  "term_id": "GO:0004984",
  "gene": "UniProtKB:Q8NGX0",
  "gene_name": "Olfactory receptor 11L1",
  "gene_symbol": "OR11L1"
}